{
  "term_label": "RNA polymerase II cis-regulatory region sequence-specific DNA binding",
  "gene": "UniProtKB:O95936",
  "gene_name": "Eomesodermin homolog",
  "term_id": "GO:0000978",
  "gene_symbol": "EOMES"
}